tail spike morphogenesis [GO:1990522] (biological process) Definition: The process in which the nematode tail spike is generated and organized. An example of this process is seen in C. elegans, where the tapered tail spike is formed during embryogenesis by a filamentous process that passes posteriorly through hyp10, the tail ventral hypodermis; the filamentous process is formed by a binucleate cell, the tail-spike cell, that subsequently undergoes programmed cell death. References: PMID:17329362, PMID:6684600 Sources: GOC:kmv Relationships: is a type of anatomical structure morphogenesis [GO:0009653]